galactosylceramide biosynthetic process [GO:0006682] (biological process) Definition: The chemical reactions and pathways resulting in the formation of galactosylceramides, any composed of a ceramide backbone covalently linked to a galactose. The galactose can be sulfated or further elongated with one more monosaccharide often a sialic acid. Relationships: is a type of GO:0006681; is a type of glycosphingolipid biosynthetic process [GO:0006688]; is a type of galactolipid biosynthetic process [GO:0019375]; is a type of ceramide biosynthetic process [GO:0046513] References: PMID:34071409 Also known as: gala-series glycosphingolipid biosynthesis, galactosylceramide anabolism, galactosylceramide biosynthesis, galactosylceramide formation, galactosylceramide synthesis